{
  "gene_name": "Sphingosine 1-phosphate receptor 1",
  "term_id": "GO:0003376",
  "term_label": "sphingosine-1-phosphate receptor signaling pathway",
  "gene_symbol": "S1PR1",
  "gene": "UniProtKB:P21453"
}